{
  "gene": "UniProtKB:O43435",
  "term_id": "GO:0006357",
  "gene_name": "T-box transcription factor TBX1",
  "gene_symbol": "TBX1",
  "term_label": "regulation of transcription by RNA polymerase II"
}